multicellular organismal-level chemical homeostasis [GO:0140962] (biological process) Sources: GOC:curators Also known as: multicellular organism level chemical homeostasis, organismal level chemical homeostasis Definition: A homeostatic process involved in the maintenance of a steady state level of a chemical within extracellular body fluids, such as blood, xylem or phloem, of a multicellular organism. This is distinct from maintenance of cellular homeostasis, which occurs within a cell. Subtypes: GO:0043129, multicellular organismal-level water homeostasis [GO:0050891], multicellular organismal-level iron ion homeostasis [GO:0060586] Relationships: is a type of multicellular organismal-level homeostasis [GO:0048871]; is a type of chemical homeostasis [GO:0048878]